{
  "gene": "UniProtKB:Q99519",
  "term_label": "membrane",
  "term_id": "GO:0016020",
  "gene_name": "Sialidase-1",
  "gene_symbol": "NEU1"
}